protein splicing [GO:0030908] (biological process) Subtypes: GO:0016539, non-intein-mediated protein splicing [GO:0030909] Definition: The post-translational removal of peptide sequences from within a protein sequence. Relationships: is a type of protein processing [GO:0016485] Sources: GOC:mah